{
  "gene_name": "G protein-regulated inducer of neurite outgrowth 2",
  "term_id": "UNKNOWN:0001",
  "gene": "UniProtKB:O60269",
  "gene_symbol": "GPRIN2",
  "term_label": "Unknown molecular function"
}